nerve growth factor production [GO:0032902] (biological process) Definition: The appearance of nerve growth factor (NGF) due to biosynthesis or secretion by cells in a neuron's target field, resulting in an increase in its intracellular or extracellular levels. Sources: GOC:ecd, GOC:mah Relationships: is a type of neurotrophin production [GO:0032898] Regulation: regulated by regulation of nerve growth factor production [GO:0032903]; negatively regulated by negative regulation of nerve growth factor production [GO:0032904] Also known as: NGF production, beta-nerve growth factor production